{
  "gene_symbol": "NOTCH2NLA",
  "gene": "UniProtKB:Q7Z3S9",
  "gene_name": "Notch homolog 2 N-terminal-like protein A",
  "term_label": "Unknown cellular component",
  "term_id": "UNKNOWN:0003"
}